{
  "term_label": "detection of chemical stimulus involved in sensory perception of smell",
  "term_id": "GO:0050911",
  "gene_name": "Olfactory receptor 10AD1",
  "gene_symbol": "OR10AD1",
  "gene": "UniProtKB:Q8NGE0"
}